{
  "term_label": "regulation of mitochondrial membrane potential",
  "gene_name": "Tumor suppressor candidate 2",
  "gene_symbol": "TUSC2",
  "gene": "UniProtKB:O75896",
  "term_id": "GO:0051881"
}